{
  "term_id": "GO:0051864",
  "gene_symbol": "RIOX2",
  "gene": "UniProtKB:Q8IUF8",
  "term_label": "histone H3K36 demethylase activity",
  "gene_name": "Ribosomal oxygenase 2"
}